{
  "gene_name": "Malonyl-CoA decarboxylase, mitochondrial",
  "term_label": "malonyl-CoA decarboxylase activity",
  "gene": "UniProtKB:O95822",
  "gene_symbol": "MLYCD",
  "term_id": "GO:0050080"
}